{
  "gene_name": "Cell adhesion molecule 4",
  "gene": "UniProtKB:Q8NFZ8",
  "term_id": "GO:0043184",
  "term_label": "vascular endothelial growth factor receptor 2 binding",
  "gene_symbol": "CADM4"
}